{
  "term_id": "GO:0005884",
  "gene_symbol": "POTEF",
  "gene": "UniProtKB:A5A3E0",
  "term_label": "actin filament",
  "gene_name": "POTE ankyrin domain family member F"
}